{
  "term_id": "GO:0071482",
  "gene": "UniProtKB:P0DN77",
  "gene_name": "Medium-wave-sensitive opsin 2",
  "gene_symbol": "OPN1MW2",
  "term_label": "cellular response to light stimulus"
}